{
  "term_label": "nucleus",
  "term_id": "GO:0005634",
  "gene_name": "tRNA (guanine-N(7)-)-methyltransferase non-catalytic subunit WDR4",
  "gene_symbol": "WDR4",
  "gene": "UniProtKB:P57081"
}